{
  "gene_name": "Protocadherin gamma-B1",
  "gene": "UniProtKB:Q9Y5G3",
  "gene_symbol": "PCDHGB1",
  "term_id": "GO:0007155",
  "term_label": "cell adhesion"
}